cadinene catabolic process [GO:1901927] (biological process) References: PMID:22867794 Sources: GOC:TermGenie Relationships: is_a sesquiterpene catabolic process [GO:0051763] Definition: The chemical reactions and pathways resulting in the breakdown of cadinene. Also known as: cadinene breakdown, cadinene catabolism, cadinene degradation